box H/ACA snoRNP complex [GO:0031429] (cellular component) Also known as: box H/ACA small nucleolar ribonucleoprotein complex, box H/ACA snoRNP pseudouridylase complex Relationships: is a type of GO:0072588; is a type of nuclear protein-containing complex [GO:0140513]; is a type of catalytic complex [GO:1902494]; is part of nucleolus [GO:0005730] References: PMID:17284456, PMID:20227365, PMID:22065625 Sources: GOC:vw Definition: A box H/ACA small nucleolar ribonucleoprotein complex located in the nucleolus that catalyzes pseudouridylation of ribosomal RNA residues. The complex is composed of four different core proteins that assemble onto a H/ACA guide RNA scaffold that identifies specific uridines in rRNA for modification during ribosome synthesis.